{
  "term_id": "GO:0019888",
  "gene_symbol": "PPP2R1B",
  "gene_name": "Serine_threonine-protein phosphatase 2A 65 kDa regulatory subunit A beta isoform",
  "term_label": "protein phosphatase regulator activity",
  "gene": "UniProtKB:P30154"
}